{
  "gene_symbol": "DNASE1L2",
  "term_label": "nucleus",
  "gene": "UniProtKB:Q92874",
  "term_id": "GO:0005634",
  "gene_name": "Deoxyribonuclease-1-like 2"
}